{
  "gene": "UniProtKB:O95255",
  "term_label": "transmembrane transport",
  "gene_name": "ATP-binding cassette sub-family C member 6",
  "term_id": "GO:0055085",
  "gene_symbol": "ABCC6"
}